{
  "gene_symbol": "L3MBTL1",
  "gene_name": "Lethal(3)malignant brain tumor-like protein 1",
  "term_label": "chromatin binding",
  "gene": "UniProtKB:Q9Y468",
  "term_id": "GO:0003682"
}